{
  "gene_name": "Vacuolar protein sorting-associated protein 26A",
  "term_id": "UNKNOWN:0001",
  "gene_symbol": "VPS26A",
  "gene": "UniProtKB:O75436",
  "term_label": "Unknown molecular function"
}